negative regulation of protein targeting to vacuolar membrane [GO:1900484] (biological process) Definition: Any process that stops, prevents or reduces the frequency, rate or extent of protein targeting to vacuolar membrane. Also known as: down regulation of protein targeting to vacuolar membrane, down-regulation of protein targeting to vacuolar membrane, downregulation of protein targeting to vacuolar membrane, inhibition of protein targeting to vacuolar membrane Relationships: is a type of negative regulation of protein targeting to membrane [GO:0090315]; is a type of negative regulation of intracellular protein transport [GO:0090317]; is a type of regulation of protein targeting to vacuolar membrane [GO:1900483]; is_a negative regulation of vacuolar transport [GO:1903336]; is_a negative regulation of protein localization to membrane [GO:1905476]; negatively regulates protein targeting to vacuolar membrane [GO:0044395] Sources: GOC:TermGenie